{
  "term_id": "GO:0003713",
  "gene": "UniProtKB:Q92793",
  "term_label": "transcription coactivator activity",
  "gene_name": "CREB-binding protein",
  "gene_symbol": "CREBBP"
}